{
  "term_id": "GO:0031461",
  "term_label": "cullin-RING ubiquitin ligase complex",
  "gene_name": "E3 ubiquitin-protein ligase RBX1",
  "gene": "UniProtKB:P62877",
  "gene_symbol": "RBX1"
}